{
  "term_label": "DNA-binding transcription factor activity, RNA polymerase II-specific",
  "gene_symbol": "CSRNP3",
  "gene": "UniProtKB:Q8WYN3",
  "term_id": "GO:0000981",
  "gene_name": "Cysteine_serine-rich nuclear protein 3"
}